{
  "gene_symbol": "RELA",
  "gene_name": "Transcription factor p65",
  "gene": "UniProtKB:Q04206",
  "term_id": "GO:0007249",
  "term_label": "canonical NF-kappaB signal transduction"
}